{
  "gene_name": "Uridine 5'-monophosphate synthase",
  "gene_symbol": "UMPS",
  "term_id": "GO:0004590",
  "gene": "UniProtKB:P11172",
  "term_label": "orotidine-5'-phosphate decarboxylase activity"
}